{
  "gene_name": "Taste receptor type 2 member 9",
  "gene_symbol": "TAS2R9",
  "term_id": "GO:0001580",
  "term_label": "detection of chemical stimulus involved in sensory perception of bitter taste",
  "gene": "UniProtKB:Q9NYW1"
}